peptidyl-aspartic acid modification [GO:0018197] (biological process) Relationships: is a type of peptidyl-amino acid modification [GO:0018193] Subtypes: N-terminal peptidyl-aspartic acid acetylation [GO:0017190], peptidyl-aspartic acid phosphorylation [GO:0018217], peptidyl-L-beta-methylthioaspartic acid biosynthetic process from peptidyl-aspartic acid [GO:0018339], peptidyl-aspartic acid hydroxylation [GO:0042264] Sources: GOC:ma Definition: The modification of peptidyl-aspartic acid.